{
  "term_label": "transcription factor TFIIA complex",
  "term_id": "GO:0005672",
  "gene": "UniProtKB:Q9UNN4",
  "gene_symbol": "GTF2A1L",
  "gene_name": "TFIIA-alpha and beta-like factor"
}